{
  "gene_name": "Metal transporter CNNM2",
  "gene_symbol": "CNNM2",
  "term_label": "plasma membrane",
  "gene": "UniProtKB:Q9H8M5",
  "term_id": "GO:0005886"
}